{
  "gene": "UniProtKB:Q9GZX6",
  "gene_name": "Interleukin-22",
  "term_label": "negative regulation of inflammatory response",
  "term_id": "GO:0050728",
  "gene_symbol": "IL22"
}